{
  "term_label": "nucleoside transmembrane transport",
  "gene_symbol": "SLC28A2",
  "term_id": "GO:1901642",
  "gene": "UniProtKB:O43868",
  "gene_name": "Sodium_nucleoside cotransporter 2"
}